{
  "gene_symbol": "SEMA6D",
  "gene_name": "Semaphorin-6D",
  "term_id": "GO:0030215",
  "term_label": "semaphorin receptor binding",
  "gene": "UniProtKB:Q8NFY4"
}